fibroblast proliferation involved in heart morphogenesis [GO:0061385] (biological process) Relationships: is a type of fibroblast proliferation [GO:0048144]; is a type of cell proliferation involved in heart morphogenesis [GO:0061323] Sources: GOC:dph Definition: The multiplication or reproduction of fibroblasts, resulting in the expansion of a fibroblast population that contributes to the shaping of the heart.